{
  "term_id": "GO:0015804",
  "term_label": "neutral amino acid transport",
  "gene_symbol": "SLC7A8",
  "gene_name": "Large neutral amino acids transporter small subunit 2",
  "gene": "UniProtKB:Q9UHI5"
}